{
  "gene": "UniProtKB:P42574",
  "gene_name": "Caspase-3",
  "term_id": "GO:0030216",
  "term_label": "keratinocyte differentiation",
  "gene_symbol": "CASP3"
}